{
  "term_label": "regulation of mRNA splicing, via spliceosome",
  "gene_name": "Serine_arginine repetitive matrix protein 1",
  "gene_symbol": "SRRM1",
  "term_id": "GO:0048024",
  "gene": "UniProtKB:Q8IYB3"
}